regulation of cholangiocyte proliferation [GO:1904054] (biological process) Definition: Any process that modulates the frequency, rate or extent of cholangiocyte proliferation. References: PMID:24434010 Sources: GOC:TermGenie, GO_REF:0000058 Also known as: regulation of hepatoblast proliferation Relationships: is a type of regulation of epithelial cell proliferation [GO:0050678]; regulates GO:1990705 Subtypes: negative regulation of cholangiocyte proliferation [GO:1904055], GO:1904056